{
  "gene_symbol": "MCMDC2",
  "gene_name": "Minichromosome maintenance domain-containing protein 2",
  "gene": "UniProtKB:Q4G0Z9",
  "term_label": "nucleus",
  "term_id": "GO:0005634"
}